regulation of cellular response to heat [GO:1900034] (biological process) Also known as: regulation of cellular response to heat stress Sources: GOC:TermGenie, GOC:yaf Relationships: is a type of regulation of cellular response to stress [GO:0080135]; regulates GO:0034605 Subtypes: negative regulation of cellular response to heat [GO:1900035], positive regulation of cellular response to heat [GO:1900036], GO:2000728 Definition: Any process that modulates the frequency, rate or extent of cellular response to heat.